{
  "term_label": "Unknown biological process",
  "gene": "UniProtKB:Q96K19",
  "term_id": "UNKNOWN:0002",
  "gene_name": "E3 ubiquitin-protein ligase RNF170",
  "gene_symbol": "RNF170"
}